{
  "term_label": "Unknown cellular component",
  "term_id": "UNKNOWN:0003",
  "gene_symbol": "PSMG3",
  "gene_name": "Proteasome assembly chaperone 3",
  "gene": "UniProtKB:Q9BT73"
}